{
  "gene_name": "Multiple C2 and transmembrane domain-containing protein 2",
  "term_id": "GO:0030672",
  "gene_symbol": "MCTP2",
  "gene": "UniProtKB:Q6DN12",
  "term_label": "synaptic vesicle membrane"
}